{
  "term_label": "cell junction",
  "term_id": "GO:0030054",
  "gene": "UniProtKB:P35609",
  "gene_name": "Alpha-actinin-2",
  "gene_symbol": "ACTN2"
}